{
  "gene_symbol": "GABRE",
  "gene_name": "Gamma-aminobutyric acid receptor subunit epsilon",
  "gene": "UniProtKB:P78334",
  "term_label": "benzodiazepine receptor activity",
  "term_id": "GO:0008503"
}